{
  "term_id": "UNKNOWN:0001",
  "gene_symbol": "FANCF",
  "gene": "UniProtKB:Q9NPI8",
  "gene_name": "Fanconi anemia group F protein",
  "term_label": "Unknown molecular function"
}